{
  "gene_symbol": "SLC16A6",
  "gene": "UniProtKB:O15403",
  "term_label": "Unknown biological process",
  "gene_name": "Monocarboxylate transporter 7",
  "term_id": "UNKNOWN:0002"
}